{
  "gene_symbol": "MBOAT2",
  "term_label": "phosphatidylcholine acyl-chain remodeling",
  "term_id": "GO:0036151",
  "gene": "UniProtKB:Q6ZWT7",
  "gene_name": "Lysophospholipid acyltransferase 2"
}